{
  "term_id": "GO:0007165",
  "gene_symbol": "MYOC",
  "gene": "UniProtKB:Q99972",
  "term_label": "signal transduction",
  "gene_name": "Myocilin"
}